{
  "gene_name": "Putative uncharacterized protein DANCR",
  "gene_symbol": "DANCR",
  "term_label": "Unknown cellular component",
  "gene": "UniProtKB:P0C864",
  "term_id": "UNKNOWN:0003"
}